{
  "term_label": "phosphatidate phosphatase activity",
  "gene_symbol": "PLPPR4",
  "gene": "UniProtKB:Q7Z2D5",
  "term_id": "GO:0008195",
  "gene_name": "Phospholipid phosphatase-related protein type 4"
}